{
  "term_id": "GO:0005794",
  "term_label": "Golgi apparatus",
  "gene": "UniProtKB:O60507",
  "gene_name": "Protein-tyrosine sulfotransferase 1",
  "gene_symbol": "TPST1"
}